CENP-T-W-S-X complex [GO:0061838] (CC) Relationships: is a type of GO:0140513; is part of chromosome, centromeric region [GO:0000775] Definition: A histone-variant containing protein complex which forms a centromere specific nucleosome-like structure, involved in centromeric chromatin organization. References: PMID:22304909, PMID:22304917